{
  "gene_symbol": "PGAP2",
  "term_id": "GO:0005789",
  "gene": "UniProtKB:Q9UHJ9",
  "term_label": "endoplasmic reticulum membrane",
  "gene_name": "Post-GPI attachment to proteins factor 2"
}